{
  "gene": "UniProtKB:P43490",
  "term_label": "Unknown cellular component",
  "gene_name": "Nicotinamide phosphoribosyltransferase",
  "term_id": "UNKNOWN:0003",
  "gene_symbol": "NAMPT"
}